{
  "gene": "UniProtKB:Q6UWR7",
  "gene_name": "Glycerophosphocholine cholinephosphodiesterase ENPP6",
  "term_label": "plasma membrane",
  "term_id": "GO:0005886",
  "gene_symbol": "ENPP6"
}